cornified envelope assembly [GO:1903575] (biological process) Note: An example of this is syntaxin 4 in PMID:22226963. References: PMID:22226963, PMID:24794495 Sources: GOC:TermGenie, GOC:pm, GO_REF:0000079 Relationships: is a type of GO:0007009; is a type of membrane assembly [GO:0071709]; has part protein-glutamine gamma-glutamyltransferase activity [GO:0003810] Definition: The aggregation, arrangement and bonding together of a set of components to form a cornified envelope. Also known as: cornified envelope formation